catalytic activity, acting on a tRNA [GO:0140101] (molecular function) Definition: Catalytic activity that acts to modify a tRNA. Relationships: is a type of catalytic activity, acting on RNA [GO:0140098] Note: Note that this term excludes activities for which a charged tRNA acts as an amino acid donor. Sources: GOC:molecular_function_refactoring, GOC:pdt Subtypes: peptidyltransferase activity [GO:0000048], tRNA 2'-phosphotransferase activity [GO:0000215], aminoacyl-tRNA deacylase activity [GO:0002161], peptidyl-tRNA hydrolase activity [GO:0004045], arginyl-tRNA--protein transferase activity [GO:0004057], L-seryl-tRNA(Sec) selenium transferase activity [GO:0004125], methionyl-tRNA formyltransferase activity [GO:0004479], tRNA-specific ribonuclease activity [GO:0004549], CCA tRNA nucleotidyltransferase activity [GO:0004810], aminoacyl-tRNA ligase activity [GO:0004812], tRNA methyltransferase activity [GO:0008175], GO:0008193, tRNA-specific adenosine deaminase activity [GO:0008251], GO:0008479, glutamyl-tRNA reductase activity [GO:0008883], GO:0008914, GO:0009022, GO:0016432, tRNA-queuosine(34) beta-mannosyltransferase activity [GO:0016438], tRNA dihydrouridine synthase activity [GO:0017150], tRNA(Ile)-lysidine synthase activity [GO:0032267], tRNA-2-methylthio-N(6)-dimethylallyladenosine(37) synthase activity [GO:0035597], GO:0035598, tRNA adenosine(64)-2'-O-ribosylphosphate transferase activity [GO:0043399], GO:0043766, tRNA 2-selenouridine synthase activity [GO:0043828], 7-cyano-7-deazaguanine tRNA-ribosyltransferase activity [GO:0043867], L-seryl-tRNA(Thr) hydrolase activity [GO:0043905], Ser(Gly)-tRNA(Ala) hydrolase activity [GO:0043908], L-seryl-tRNA(Sec) kinase activity [GO:0043915], GO:0045301, GO:0050566, glutaminyl-tRNA synthase (glutamine-hydrolyzing) activity [GO:0050567], GO:0051075, tRNA cytidine N4-acetyltransferase activity [GO:0051392], tRNA dimethylallyltransferase activity [GO:0052381], CC tRNA cytidylyltransferase activity [GO:0052927], ATP:3'-cytidine-cytidine-tRNA adenylyltransferase activity [GO:0052929], tRNA threonylcarbamoyladenosine dehydratase [GO:0061503], GO:0061708, tRNA N(6)-L-threonylcarbamoyladenine synthase activity [GO:0061711], GO:0098620, O-phosphoseryl-tRNA(Sec) selenium transferase activity [GO:0098621], tRNA-4-demethylwyosine synthase activity [GO:0102521], tRNA 4-demethylwyosine alpha-amino-alpha-carboxypropyltransferase activity [GO:0102522], tRNA(Phe) (7-(3-amino-3-carboxypropyl)wyosine37-C2)-hydroxylase activity [GO:0102524], tRNA-uridine 2-sulfurtransferase activity [GO:0103016], tRNA pseudouridine synthase activity [GO:0106029], GO:0106261, tRNA-uracil-4 sulfurtransferase activity [GO:0140741], GO:0141125, CCACCA tRNA nucleotidyltransferase activity [GO:0160016], tRNA 5-taurinomethyluridine synthase activity [GO:0160236], 2-oxoglutarate-dependent tRNA 5-methylcytidine formyltransferase activity [GO:0160290], tRNA demethylase activity [GO:1990984]